2-hydroxylaminobenzoate reductase activity [GO:0034557] (molecular function) Relationships: is a type of oxidoreductase activity, acting on the CH-NH2 group of donors [GO:0016638] Definition: Catalysis of the reaction: 2-hydroxylaminobenzoate + NAD(P)H = anthranilate + NAD(P)+ + H2O. Also known as: o-hydroxylaminobenzoate nitroreductase activity Sources: MetaCyc:RXN-8848